{
  "term_label": "regulation of intracellular signal transduction",
  "gene_name": "Ras GTPase-activating protein 4",
  "gene_symbol": "RASA4",
  "gene": "UniProtKB:O43374",
  "term_id": "GO:1902531"
}